{
  "gene": "UniProtKB:Q6P9B6",
  "term_id": "UNKNOWN:0001",
  "gene_symbol": "MEAK7",
  "term_label": "Unknown molecular function",
  "gene_name": "MTOR-associated protein MEAK7"
}